propionate CoA-transferase activity [GO:0018729] (molecular function) Sources: EC:2.8.3.1 Relationships: is a type of CoA-transferase activity [GO:0008410] Also known as: acetyl-CoA:propanoate CoA-transferase activity, propionate coenzyme A-transferase activity, propionate-CoA:lactoyl-CoA transferase activity, propionyl CoA:acetate CoA transferase activity, propionyl-CoA transferase activity Definition: Catalysis of the reaction: acetyl-CoA + propanoate = acetate + propanoyl-CoA.